{
  "gene": "UniProtKB:Q9Y282",
  "gene_symbol": "ERGIC3",
  "term_label": "endoplasmic reticulum membrane",
  "term_id": "GO:0005789",
  "gene_name": "Endoplasmic reticulum-Golgi intermediate compartment protein 3"
}